{
  "gene": "UniProtKB:Q8N3A8",
  "gene_symbol": "PARP8",
  "term_label": "NAD+ poly-ADP-ribosyltransferase activity",
  "gene_name": "Protein mono-ADP-ribosyltransferase PARP8",
  "term_id": "GO:0003950"
}